{
  "gene_name": "Neuromedin-B receptor",
  "gene_symbol": "NMBR",
  "gene": "UniProtKB:P28336",
  "term_id": "GO:0005886",
  "term_label": "plasma membrane"
}